{
  "gene": "UniProtKB:Q96I34",
  "term_label": "myosin phosphatase regulator activity",
  "gene_name": "Protein phosphatase 1 regulatory subunit 16A",
  "term_id": "GO:0017020",
  "gene_symbol": "PPP1R16A"
}